{
  "gene": "UniProtKB:Q96SL1",
  "term_id": "UNKNOWN:0002",
  "term_label": "Unknown biological process",
  "gene_name": "Solute carrier family 49 member 4",
  "gene_symbol": "SLC49A4"
}